{
  "gene_symbol": "CSNK1E",
  "gene": "UniProtKB:P49674",
  "term_id": "GO:0004674",
  "term_label": "protein serine/threonine kinase activity",
  "gene_name": "Casein kinase I isoform epsilon"
}